{
  "gene_symbol": "PTK7",
  "term_label": "axon",
  "term_id": "GO:0030424",
  "gene": "UniProtKB:Q13308",
  "gene_name": "Inactive tyrosine-protein kinase 7"
}